{
  "term_id": "GO:0032502",
  "term_label": "developmental process",
  "gene_name": "Probable RNA polymerase II nuclear localization protein SLC7A6OS",
  "gene_symbol": "SLC7A6OS",
  "gene": "UniProtKB:Q96CW6"
}